negative regulation of ubiquinone biosynthetic process [GO:1904774] (biological process) Definition: Any process that stops, prevents or reduces the frequency, rate or extent of ubiquinone biosynthetic process. References: PMID:8125303 Sources: GOC:TermGenie, GO_REF:0000058 Also known as: down regulation of coenzyme Q biosynthesis, down regulation of coenzyme Q biosynthetic process, down regulation of ubiquinone anabolism, down regulation of ubiquinone biosynthesis, down regulation of ubiquinone biosynthetic process, down regulation of ubiquinone formation, down regulation of ubiquinone synthesis, down-regulation of coenzyme Q biosynthesis, down-regulation of coenzyme Q biosynthetic process, down-regulation of ubiquinone anabolism, down-regulation of ubiquinone biosynthesis, down-regulation of ubiquinone biosynthetic process, down-regulation of ubiquinone formation, down-regulation of ubiquinone synthesis, downregulation of coenzyme Q biosynthesis, downregulation of coenzyme Q biosynthetic process, downregulation of ubiquinone anabolism, downregulation of ubiquinone biosynthesis, downregulation of ubiquinone biosynthetic process, downregulation of ubiquinone formation, downregulation of ubiquinone synthesis, negative regulation of coenzyme Q biosynthesis, negative regulation of coenzyme Q biosynthetic process, negative regulation of ubiquinone anabolism, negative regulation of ubiquinone biosynthesis, negative regulation of ubiquinone formation, negative regulation of ubiquinone synthesis, down regulation of coenzyme Q10 biosynthesis, down regulation of coenzyme Q10 biosynthetic process, down regulation of coenzyme Q6 biosynthesis, down regulation of coenzyme Q6 biosynthetic process, down regulation of coenzyme Q8 biosynthesis, down regulation of coenzyme Q8 biosynthetic process, down regulation of coenzyme Q9 biosynthesis, down regulation of coenzyme Q9 biosynthetic process, down-regulation of coenzyme Q10 biosynthesis, down-regulation of coenzyme Q10 biosynthetic process, down-regulation of coenzyme Q6 biosynthesis, down-regulation of coenzyme Q6 biosynthetic process, down-regulation of coenzyme Q8 biosynthesis, down-regulation of coenzyme Q8 biosynthetic process, down-regulation of coenzyme Q9 biosynthesis, down-regulation of coenzyme Q9 biosynthetic process, downregulation of coenzyme Q10 biosynthesis, downregulation of coenzyme Q10 biosynthetic process, downregulation of coenzyme Q6 biosynthesis, downregulation of coenzyme Q6 biosynthetic process, downregulation of coenzyme Q8 biosynthesis, downregulation of coenzyme Q8 biosynthetic process, downregulation of coenzyme Q9 biosynthesis, downregulation of coenzyme Q9 biosynthetic process, inhibition of coenzyme Q biosynthesis, inhibition of coenzyme Q biosynthetic process, inhibition of coenzyme Q10 biosynthesis, inhibition of coenzyme Q10 biosynthetic process, inhibition of coenzyme Q6 biosynthesis, inhibition of coenzyme Q6 biosynthetic process, inhibition of coenzyme Q8 biosynthesis, inhibition of coenzyme Q8 biosynthetic process, inhibition of coenzyme Q9 biosynthesis, inhibition of coenzyme Q9 biosynthetic process, inhibition of ubiquinone anabolism, inhibition of ubiquinone biosynthesis, inhibition of ubiquinone biosynthetic process, inhibition of ubiquinone formation, inhibition of ubiquinone synthesis, negative regulation of coenzyme Q10 biosynthesis, negative regulation of coenzyme Q10 biosynthetic process, negative regulation of coenzyme Q6 biosynthesis, negative regulation of coenzyme Q6 biosynthetic process, negative regulation of coenzyme Q8 biosynthesis, negative regulation of coenzyme Q8 biosynthetic process, negative regulation of coenzyme Q9 biosynthesis, negative regulation of coenzyme Q9 biosynthetic process Relationships: is a type of negative regulation of biosynthetic process [GO:0009890]; is a type of GO:0010795; is a type of GO:0062014; negatively regulates ubiquinone biosynthetic process [GO:0006744]